tRNA dihydrouridine synthase activity [GO:0017150] (molecular function) Subtypes: tRNA-dihydrouridine16 synthase activity [GO:0102262], tRNA-dihydrouridine17 synthase activity [GO:0102263], tRNA-dihydrouridine20 synthase activity [GO:0102264], tRNA-dihydrouridine47 synthase activity [GO:0102265], tRNA-dihydrouridine20a synthase activity [GO:0102266], tRNA-dihydrouridine20b synthase activity [GO:0102267] Relationships: is a type of RNA dihydrouridine synthase activity [GO:0106413]; is a type of GO:0140101; is part of tRNA dihydrouridine synthesis [GO:0002943] References: PMID:11983710, PMID:22123979 Definition: Catalysis of the reaction: a 5,6-dihydrouridine in tRNA + NAD(P)+ = a uridine in tRNA + H+ + NAD(P)H.